lysozyme inhibitor activity [GO:0060241] (molecular function) Relationships: is a type of enzyme inhibitor activity [GO:0004857]; negatively regulates lysozyme activity [GO:0003796] Sources: GOC:dph Definition: Binds to and stops, prevents or reduces the activity of lysozyme.